production of molecular mediator involved in inflammatory response [GO:0002532] (biological process) Sources: GOC:add, GOC:dph, GOC:tb, ISBN:0781735149 Relationships: is a type of multicellular organismal process [GO:0032501]; is part of GO:0006954 Also known as: production of molecular mediator involved in acute inflammatory response, production of cellular mediator of acute inflammation Subtypes: histamine production involved in inflammatory response [GO:0002349], serotonin production involved in inflammatory response [GO:0002351], GO:0002391, lysosomal enzyme production involved in inflammatory response [GO:0002393], cytokine production involved in inflammatory response [GO:0002534], GO:0002536, nitric oxide production involved in inflammatory response [GO:0002537], arachidonate metabolite production involved in inflammatory response [GO:0002538] Definition: The synthesis or release of any molecular mediator of the inflammatory response following an inflammatory stimulus, resulting in an increase in its intracellular or extracellular levels.